{
  "gene": "UniProtKB:Q86XP3",
  "term_label": "Unknown biological process",
  "term_id": "UNKNOWN:0002",
  "gene_symbol": "DDX42",
  "gene_name": "ATP-dependent RNA helicase DDX42"
}